positive regulation of asymmetric protein localization involved in cell fate determination [GO:1904787] (biological process) Definition: Any process that activates or increases the frequency, rate or extent of asymmetric protein localization involved in cell fate determination. Note: wrm-1 in C. Elegans (Q10953) in PMID:17476329 (IMP) References: PMID:17476329 Sources: GOC:TermGenie, GO_REF:0000058 Also known as: positive regulation of asymmetric protein localisation involved in cell fate determination, positive regulation of asymmetric protein localization involved in cell fate commitment, positive regulation of asymmetric protein localization resulting in cell fate commitment, positive regulation of cell fate commitment, asymmetric protein localization, up regulation of asymmetric protein localisation involved in cell fate determination, up regulation of asymmetric protein localization involved in cell fate commitment, up regulation of asymmetric protein localization involved in cell fate determination, up regulation of asymmetric protein localization resulting in cell fate commitment, up regulation of cell fate commitment, asymmetric protein localization, up-regulation of asymmetric protein localisation involved in cell fate determination, up-regulation of asymmetric protein localization involved in cell fate commitment, up-regulation of asymmetric protein localization involved in cell fate determination, up-regulation of asymmetric protein localization resulting in cell fate commitment, up-regulation of cell fate commitment, asymmetric protein localization, upregulation of asymmetric protein localisation involved in cell fate determination, upregulation of asymmetric protein localization involved in cell fate commitment, upregulation of asymmetric protein localization involved in cell fate determination, upregulation of asymmetric protein localization resulting in cell fate commitment, upregulation of cell fate commitment, asymmetric protein localization, activation of asymmetric protein localisation involved in cell fate determination, activation of asymmetric protein localization involved in cell fate commitment, activation of asymmetric protein localization involved in cell fate determination, activation of asymmetric protein localization resulting in cell fate commitment, activation of cell fate commitment, asymmetric protein localization Relationships: is a type of GO:1903829; is_a GO:1904785; positively regulates asymmetric protein localization involved in cell fate determination [GO:0045167]